{
  "term_label": "actin filament",
  "term_id": "GO:0005884",
  "gene_name": "Tropomyosin beta chain",
  "gene_symbol": "TPM2",
  "gene": "UniProtKB:P07951"
}